{
  "term_id": "UNKNOWN:0003",
  "term_label": "Unknown cellular component",
  "gene": "UniProtKB:Q12901",
  "gene_symbol": "ZNF155",
  "gene_name": "Zinc finger protein 155"
}